{
  "term_label": "ammonium channel activity",
  "gene": "UniProtKB:Q02094",
  "gene_name": "Ammonium transporter Rh type A",
  "term_id": "GO:0008519",
  "gene_symbol": "RHAG"
}